{
  "term_label": "Unknown cellular component",
  "gene_symbol": "NPIPA1",
  "gene_name": "Nuclear pore complex-interacting protein family member A1",
  "gene": "UniProtKB:Q9UND3",
  "term_id": "UNKNOWN:0003"
}